{
  "term_id": "GO:0098609",
  "gene": "UniProtKB:P17301",
  "gene_symbol": "ITGA2",
  "gene_name": "Integrin alpha-2",
  "term_label": "cell-cell adhesion"
}